positive regulation of cytokinesis, site selection [GO:2000076] (biological process) Sources: GOC:mtg_cell_cycle, GOC:obol Also known as: positive regulation of site selection involved in cell cycle cytokinesis Relationships: is a type of positive regulation of cytokinesis [GO:0032467]; is a type of regulation of cytokinesis, site selection [GO:2000073]; positively regulates cytokinesis, division site positioning [GO:0007105] Definition: Any process that activates or increases the frequency, rate or extent of site selection that occurs as part of cytokinesis. Subtypes: positive regulation of mitotic cytokinesis, division site positioning [GO:1903617]